{
  "gene_name": "C-type lectin domain family 4 member K",
  "gene_symbol": "CD207",
  "term_label": "pattern recognition receptor activity",
  "gene": "UniProtKB:Q9UJ71",
  "term_id": "GO:0038187"
}